{
  "term_label": "CCR4-NOT core complex",
  "gene_name": "CCR4-NOT transcription complex subunit 9",
  "term_id": "GO:0030015",
  "gene_symbol": "CNOT9",
  "gene": "UniProtKB:Q92600"
}